{
  "term_id": "GO:0098793",
  "gene_name": "Synaptojanin-1",
  "gene_symbol": "SYNJ1",
  "gene": "UniProtKB:O43426",
  "term_label": "presynapse"
}